choline binding [GO:0033265] (molecular function) Relationships: is a type of GO:0043169 Sources: GOC:mlg Definition: Binding to choline, the amine 2-hydroxy-N,N,N-trimethylethanaminium.